{
  "gene_name": "Moesin",
  "term_label": "actin binding",
  "gene_symbol": "MSN",
  "term_id": "GO:0003779",
  "gene": "UniProtKB:P26038"
}